{
  "gene_name": "Immediate early response gene 5-like protein",
  "term_id": "UNKNOWN:0003",
  "gene": "UniProtKB:Q5T953",
  "term_label": "Unknown cellular component",
  "gene_symbol": "IER5L"
}